phenylmercury acetate catabolic process [GO:0019506] (BP) Definition: The chemical reactions and pathways resulting in the breakdown of phenylmercury acetate, an organomercurial compound composed of a mercury atom attached to a benzene ring and an acetate group. Relationships: is a type of organometal metabolic process [GO:0018942]; is a type of GO:0042178; is a type of benzene-containing compound metabolic process [GO:0042537] Also known as: phenylmercury acetate breakdown, phenylmercury acetate catabolism, phenylmercury acetate degradation Sources: GOC:ai